{
  "gene_symbol": "TTLL4",
  "gene_name": "Tubulin monoglutamylase TTLL4",
  "term_label": "microtubule cytoskeleton organization",
  "term_id": "GO:0000226",
  "gene": "UniProtKB:Q14679"
}